positive regulation of ruffle assembly [GO:1900029] (biological process) Sources: GOC:TermGenie, GOC:yaf Also known as: positive regulation of membrane ruffle formation, positive regulation of membrane ruffling, up regulation of membrane ruffle formation, up regulation of membrane ruffling, up regulation of ruffle assembly Definition: Any process that activates or increases the frequency, rate or extent of ruffle assembly. Relationships: is a type of positive regulation of plasma membrane bounded cell projection assembly [GO:0120034]; is a type of regulation of ruffle assembly [GO:1900027]; positively regulates GO:0097178